{
  "gene_symbol": "RAB43",
  "term_label": "autophagosome assembly",
  "gene_name": "Ras-related protein Rab-43",
  "gene": "UniProtKB:Q86YS6",
  "term_id": "GO:0000045"
}